{
  "gene_name": "Small ribosomal subunit protein eS4, X isoform",
  "term_label": "cytosolic small ribosomal subunit",
  "term_id": "GO:0022627",
  "gene_symbol": "RPS4X",
  "gene": "UniProtKB:P62701"
}